{
  "gene_symbol": "SLC47A1",
  "gene_name": "Multidrug and toxin extrusion protein 1",
  "term_label": "organic cation transport",
  "gene": "UniProtKB:Q96FL8",
  "term_id": "GO:0015695"
}